{
  "term_id": "GO:0005737",
  "term_label": "cytoplasm",
  "gene_symbol": "DSP",
  "gene": "UniProtKB:P15924",
  "gene_name": "Desmoplakin"
}